{
  "gene": "UniProtKB:O00180",
  "gene_name": "Potassium channel subfamily K member 1",
  "term_label": "potassium ion transmembrane transport",
  "term_id": "GO:0071805",
  "gene_symbol": "KCNK1"
}